telomerase RNA binding [GO:0070034] (molecular function) References: PMID:16884717 Sources: GOC:krc Relationships: is a type of GO:0003723 Definition: Binding to the telomerase RNA template. Also known as: TERC binding